negative regulation of urine volume [GO:0035811] (biological process) Relationships: is a type of regulation of urine volume [GO:0035809] Also known as: antidiuresis, decrease in urine flow, reduction of urinary volume Subtypes: renal water retention [GO:0003092] Sources: GOC:mtg_25march11, GOC:yaf Definition: Any process that decreases the amount of urine excreted from the body over a unit of time.